{
  "gene_name": "Fatty acid-binding protein 5",
  "term_id": "GO:0005504",
  "term_label": "fatty acid binding",
  "gene_symbol": "FABP5",
  "gene": "UniProtKB:Q01469"
}